{
  "term_label": "Unknown molecular function",
  "term_id": "UNKNOWN:0001",
  "gene": "UniProtKB:P35219",
  "gene_name": "Carbonic anhydrase-related protein",
  "gene_symbol": "CA8"
}